{
  "gene": "UniProtKB:Q9BPX5",
  "term_id": "GO:0016477",
  "gene_name": "Actin-related protein 2_3 complex subunit 5-like protein",
  "term_label": "cell migration",
  "gene_symbol": "ARPC5L"
}